siRNA-mediated long-distance post-transcriptional gene silencing [GO:0010495] (biological process) References: PMID:11590235, PMID:17785412 Sources: GOC:dph, GOC:tb Relationships: is a type of GO:0090625 Definition: An siRNA-mediated posttranscriptional gene silencing pathway in which small interfering RNAs (siRNAs) direct the cleavage of target mRNAs, and in which the silencing signal originates in one tissue and occurs in a different tissue. Also known as: long-distance posttranscriptional gene silencing, long-distance propagation of posttranscriptional gene silencing, siRNA-mediated long-distance posttranscriptional gene silencing